{
  "term_id": "UNKNOWN:0001",
  "gene_name": "Ras association domain-containing protein 3",
  "term_label": "Unknown molecular function",
  "gene": "UniProtKB:Q86WH2",
  "gene_symbol": "RASSF3"
}